{
  "term_id": "UNKNOWN:0003",
  "gene": "UniProtKB:Q9H4F1",
  "term_label": "Unknown cellular component",
  "gene_name": "Alpha-N-acetyl-neuraminyl-2,3-beta-galactosyl-1,3-N-acetyl-galactosaminide alpha-2,6-sialyltransferase",
  "gene_symbol": "ST6GALNAC4"
}